{
  "gene": "UniProtKB:P48201",
  "gene_symbol": "ATP5MC3",
  "term_id": "GO:0015986",
  "gene_name": "ATP synthase F(0) complex subunit C3, mitochondrial",
  "term_label": "proton motive force-driven ATP synthesis"
}